{
  "gene_symbol": "LAIR1",
  "gene": "UniProtKB:Q6GTX8",
  "term_id": "GO:0005886",
  "gene_name": "Leukocyte-associated immunoglobulin-like receptor 1",
  "term_label": "plasma membrane"
}